{
  "gene_name": "tRNA pseudouridine(38_39) synthase",
  "term_label": "pseudouridine synthase activity",
  "gene_symbol": "PUS3",
  "term_id": "GO:0009982",
  "gene": "UniProtKB:Q9BZE2"
}